semaphorin-plexin signaling pathway involved in regulation of photoreceptor cell axon guidance [GO:2000305] (biological process) Definition: Any semaphorin-plexin signaling pathway that is involved in regulation of photoreceptor cell axon guidance. Relationships: is a type of GO:0071526; is part of regulation of photoreceptor cell axon guidance [GO:2000289] Sources: GOC:obol Also known as: semaphorin-plexin signaling pathway of regulation of photoreceptor cell axon guidance, semaphorin-plexin signaling pathway of regulation of photoreceptor cell axon pathfinding, semaphorin-plexin signalling pathway of regulation of photoreceptor cell axon guidance, semaphorin-plexin signalling pathway of regulation of photoreceptor cell axon pathfinding